{
  "term_label": "Cul4-RING E3 ubiquitin ligase complex",
  "gene": "UniProtKB:P0C7V8",
  "term_id": "GO:0080008",
  "gene_name": "DDB1- and CUL4-associated factor 8-like protein 2",
  "gene_symbol": "DCAF8L2"
}